parasexual reproduction with cellular fusion [GO:1990277] (biological process) References: PMID:26210747 Sources: GOC:di Also known as: mating, parasexual conjugation with cellular fusion Relationships: is a type of reproductive process [GO:0022414]; has part GO:0140253 Definition: A type of reproduction in which new individuals are produced from two individuals, with the fusion of two somatic cells.